{
  "gene": "UniProtKB:O15041",
  "gene_symbol": "SEMA3E",
  "gene_name": "Semaphorin-3E",
  "term_label": "semaphorin receptor binding",
  "term_id": "GO:0030215"
}